{
  "gene_name": "Anaphase-promoting complex subunit 11",
  "term_id": "GO:0045842",
  "gene_symbol": "ANAPC11",
  "gene": "UniProtKB:Q9NYG5",
  "term_label": "positive regulation of mitotic metaphase/anaphase transition"
}